{
  "gene_name": "CTD small phosphatase-like protein 2",
  "term_label": "Unknown cellular component",
  "gene_symbol": "CTDSPL2",
  "gene": "UniProtKB:Q05D32",
  "term_id": "UNKNOWN:0003"
}